{
  "gene": "UniProtKB:Q9Y6N1",
  "gene_symbol": "COX11",
  "term_id": "GO:0005743",
  "gene_name": "Cytochrome c oxidase assembly protein COX11, mitochondrial",
  "term_label": "mitochondrial inner membrane"
}